{
  "term_label": "Unknown biological process",
  "gene": "UniProtKB:Q12805",
  "gene_symbol": "EFEMP1",
  "gene_name": "EGF-containing fibulin-like extracellular matrix protein 1",
  "term_id": "UNKNOWN:0002"
}